{
  "gene_symbol": "ANKRD26",
  "term_id": "UNKNOWN:0002",
  "term_label": "Unknown biological process",
  "gene_name": "Ankyrin repeat domain-containing protein 26",
  "gene": "UniProtKB:Q9UPS8"
}